{
  "gene_symbol": "AKAP14",
  "gene": "UniProtKB:Q86UN6",
  "term_id": "GO:0005952",
  "gene_name": "A-kinase anchor protein 14",
  "term_label": "cAMP-dependent protein kinase complex"
}